{
  "gene_symbol": "MAP3K6",
  "gene": "UniProtKB:O95382",
  "gene_name": "Mitogen-activated protein kinase kinase kinase 6",
  "term_id": "GO:0007254",
  "term_label": "JNK cascade"
}